{
  "gene_name": "Endoplasmic reticulum aminopeptidase 2",
  "gene_symbol": "ERAP2",
  "term_label": "metalloaminopeptidase activity",
  "gene": "UniProtKB:Q6P179",
  "term_id": "GO:0070006"
}